{
  "gene": "UniProtKB:Q07326",
  "gene_symbol": "PIGF",
  "term_label": "GPI anchor biosynthetic process",
  "gene_name": "Phosphatidylinositol-glycan biosynthesis class F protein",
  "term_id": "GO:0006506"
}